peroxisome membrane biogenesis [GO:0016557] (biological process) Definition: The process in which a peroxisome membrane is synthesized, aggregates, and bonds together. Relationships: is a type of membrane biogenesis [GO:0044091]; is part of GO:0007031 Sources: GOC:mah